{
  "gene_name": "Collagen alpha-1(XXIII) chain",
  "gene": "UniProtKB:Q86Y22",
  "term_id": "GO:0030020",
  "term_label": "extracellular matrix structural constituent conferring tensile strength",
  "gene_symbol": "COL23A1"
}